{
  "gene_symbol": "ORM1",
  "term_label": "Unknown biological process",
  "term_id": "UNKNOWN:0002",
  "gene_name": "Alpha-1-acid glycoprotein 1",
  "gene": "UniProtKB:P02763"
}